{
  "term_label": "proton-transporting ATPase activity, rotational mechanism",
  "gene_name": "V-type proton ATPase catalytic subunit A",
  "gene_symbol": "ATP6V1A",
  "term_id": "GO:0046961",
  "gene": "UniProtKB:P38606"
}